symbiont-mediated activation of host autophagy [GO:0039520] (biological process) Subtypes: symbiont-mediated activation of host reticulophagy [GO:0140883] Relationships: is a type of symbiont-mediated perturbation of host autophagy [GO:0075071] Also known as: positive regulation by virus of host autophagy, activation of host autophagy by virus, induction by virus of host autophagy, autophagy of host cells involved in interaction with symbiont Sources: GOC:bf, GOC:sp, VZ:846 Definition: A process in which a symbiont initiates, promotes, or enhances the normal execution of autophagy in the host cell. The host is defined as the larger of the organisms involved in a symbiotic interaction. For example, some viruses are able to activate host autophagy as a cellular survival mechanism, hence delaying or inhibiting apoptosis.